response to host oxygen tension environment [GO:0075138] (biological process) Sources: GOC:pamgo_curators Relationships: is a type of response to host [GO:0075136] Also known as: response of symbiont to host oxygen tension environment Definition: Any process that results in a change in state or activity of the symbiont or its cell (in terms of movement, secretion, enzyme production, gene expression, etc.) as a result of detecting oxygen tension in the host organism. The host is defined as the larger of the organisms involved in a symbiotic interaction. Note: Note that this term is used to annotate gene products of the symbiont.